S-adenosylmethionine-homocysteine S-methyltransferase activity [GO:0008898] (molecular function) Sources: RHEA:21820 Definition: Catalysis of the reaction: S-adenosyl-L-methionine + L-homocysteine = S-adenosyl-L-homocysteine + L-methionine. Also known as: L-homocysteine S-methyltransferase activity, S-adenosyl-L-methionine:L-homocysteine S-methyltransferase activity, S-adenosyl-L-methionine:L-homocysteine methyltransferase activity, S-adenosylmethionine homocysteine transmethylase activity, S-adenosylmethionine-homocysteine transmethylase activity, S-adenosylmethionine:homocysteine methyltransferase activity, adenosylmethionine transmethylase activity, adenosylmethionine:homocysteine methyltransferase activity, homocysteine methyltransferase activity, homocysteine transmethylase activity Relationships: is a type of S-methyltransferase activity [GO:0008172]; is a type of S-adenosylmethionine-dependent methyltransferase activity [GO:0008757]